2-methylbut-2-enoyl-CoA(4-) catabolic process [GO:1902193] (biological process) Definition: The chemical reactions and pathways resulting in the breakdown of 2-methylbut-2-enoyl-CoA(4-). References: PMID:15574432 Sources: GOC:TermGenie Also known as: 2-methylbut-2-enoyl-CoA(4-) breakdown, 2-methylbut-2-enoyl-CoA(4-) catabolism, 2-methylbut-2-enoyl-CoA(4-) degradation Relationships: is a type of fatty-acyl-CoA catabolic process [GO:0036115]; is a type of GO:1902192